{
  "gene_symbol": "ZFP36",
  "gene_name": "mRNA decay activator protein ZFP36",
  "term_label": "mRNA regulatory element binding translation repressor activity",
  "term_id": "GO:0000900",
  "gene": "UniProtKB:P26651"
}